{
  "gene_name": "Small ribosomal subunit protein eS17",
  "gene": "UniProtKB:P08708",
  "gene_symbol": "RPS17",
  "term_label": "structural constituent of ribosome",
  "term_id": "GO:0003735"
}